{
  "gene_symbol": "FAM90A14",
  "term_label": "Unknown cellular component",
  "term_id": "UNKNOWN:0003",
  "gene_name": "Putative protein FAM90A14",
  "gene": "UniProtKB:P0C7W9"
}